beta-gentiobiose beta-glucosidase activity [GO:0080083] (molecular function) References: PMID:15604686 Definition: Catalysis of the hydrolysis of glucosidic link in beta-gentiobiose. Relationships: is a type of GO:0008422